BH domain binding [GO:0051400] (molecular function) Definition: Binding to a Bcl-2 homology (BH) protein domain. Bcl-2-related proteins share homology in one to four conserved regions designated the Bcl-2 homology (BH) domains BH1, BH2, BH3 and BH4. These domains contribute at multiple levels to the function of these proteins in cell death and survival. Anti-apoptotic members of the Bcl-2 family have four BH domains (BH1-BH4). Pro-apoptotic members have fewer BH domains. References: PMID:11048732, PMID:12133724, PMID:9020082, PMID:9704409 Subtypes: BH1 domain binding [GO:0051432], BH2 domain binding [GO:0051433], BH3 domain binding [GO:0051434], GO:0051435 Relationships: is a type of protein domain specific binding [GO:0019904] Also known as: Bcl-2 homology domain binding